{
  "gene": "UniProtKB:Q6IEE7",
  "term_id": "GO:0016020",
  "gene_name": "Transmembrane protein 132E",
  "term_label": "membrane",
  "gene_symbol": "TMEM132E"
}